{
  "term_label": "positive regulation of immature T cell proliferation in thymus",
  "gene_symbol": "IL1B",
  "gene_name": "Interleukin-1 beta",
  "term_id": "GO:0033092",
  "gene": "UniProtKB:P01584"
}